{
  "term_id": "GO:0006805",
  "gene": "UniProtKB:Q99518",
  "term_label": "xenobiotic metabolic process",
  "gene_name": "Flavin-containing monooxygenase 2",
  "gene_symbol": "FMO2"
}